{
  "term_id": "GO:0000981",
  "gene_symbol": "ERG",
  "gene_name": "Transcriptional regulator ERG",
  "term_label": "DNA-binding transcription factor activity, RNA polymerase II-specific",
  "gene": "UniProtKB:P11308"
}